{
  "gene": "UniProtKB:P43307",
  "gene_name": "Translocon-associated protein subunit alpha",
  "gene_symbol": "SSR1",
  "term_label": "endoplasmic reticulum",
  "term_id": "GO:0005783"
}